{
  "term_label": "plasma membrane",
  "gene": "UniProtKB:Q6NSJ5",
  "term_id": "GO:0005886",
  "gene_name": "Volume-regulated anion channel subunit LRRC8E",
  "gene_symbol": "LRRC8E"
}